{
  "gene": "UniProtKB:P54619",
  "gene_name": "5'-AMP-activated protein kinase subunit gamma-1",
  "term_label": "nucleus",
  "term_id": "GO:0005634",
  "gene_symbol": "PRKAG1"
}